{
  "term_id": "GO:0005634",
  "term_label": "nucleus",
  "gene": "UniProtKB:Q7L5Y6",
  "gene_symbol": "DET1",
  "gene_name": "DET1 homolog"
}